{
  "gene_symbol": "TRIM39",
  "term_label": "regulation of gene expression",
  "gene": "UniProtKB:Q9HCM9",
  "gene_name": "E3 ubiquitin-protein ligase TRIM39",
  "term_id": "GO:0010468"
}